negative regulation of autophagic cell death [GO:1904093] (biological process) References: PMID:25736836 Sources: GOC:TermGenie, GOC:bhm, GO_REF:0000058 Also known as: down regulation of autophagic cell death, down regulation of programmed cell death by macroautophagy, down-regulation of autophagic cell death, down-regulation of programmed cell death by macroautophagy, downregulation of autophagic cell death, downregulation of programmed cell death by macroautophagy, negative regulation of programmed cell death by macroautophagy, inhibition of autophagic cell death, inhibition of programmed cell death by macroautophagy, down regulation of type II programmed cell death, down-regulation of type II programmed cell death, downregulation of type II programmed cell death, inhibition of type II programmed cell death, negative regulation of type II programmed cell death Relationships: is a type of GO:0043069; is a type of GO:1904092; negatively regulates GO:0048102 Definition: Any process that stops, prevents or reduces the frequency, rate or extent of autophagic cell death.